{
  "gene_symbol": "TASP1",
  "gene_name": "Threonine aspartase 1",
  "term_id": "GO:0051604",
  "term_label": "protein maturation",
  "gene": "UniProtKB:Q9H6P5"
}